coenzyme A transmembrane transporter activity [GO:0015228] (MF) Definition: Enables the transfer of coenzyme A from one side of a membrane to the other. Coenzyme A, 3'-phosphoadenosine-(5')diphospho(4')pantatheine, is an acyl carrier in many acylation and acyl-transfer reactions in which the intermediate is a thiol ester. Sources: GOC:ai Also known as: coenzyme A transporter activity Relationships: is a type of organophosphate ester transmembrane transporter activity [GO:0015605]; is a type of nucleobase-containing compound transmembrane transporter activity [GO:0015932]; is a type of amide transmembrane transporter activity [GO:0042887]; is a type of sulfur compound transmembrane transporter activity [GO:1901682]; is part of GO:0035349 Subtypes: GO:0015325